regulation of osteoblast proliferation [GO:0033688] (biological process) Subtypes: negative regulation of osteoblast proliferation [GO:0033689], positive regulation of osteoblast proliferation [GO:0033690] Relationships: is a type of regulation of cell population proliferation [GO:0042127]; regulates osteoblast proliferation [GO:0033687] Sources: GOC:mah Definition: Any process that modulates the frequency, rate or extent of osteoblast proliferation.